{
  "term_id": "GO:0019677",
  "gene_name": "NAD-capped RNA hydrolase NUDT12",
  "term_label": "NAD+ catabolic process",
  "gene_symbol": "NUDT12",
  "gene": "UniProtKB:Q9BQG2"
}